{
  "gene_symbol": "RER1",
  "term_label": "retrograde vesicle-mediated transport, Golgi to endoplasmic reticulum",
  "gene": "UniProtKB:O15258",
  "gene_name": "Protein RER1",
  "term_id": "GO:0006890"
}